{
  "gene": "UniProtKB:O75251",
  "term_label": "mitochondrial respiratory chain complex I assembly",
  "gene_symbol": "NDUFS7",
  "gene_name": "NADH dehydrogenase [ubiquinone] iron-sulfur protein 7, mitochondrial",
  "term_id": "GO:0032981"
}